{
  "gene_symbol": "DHX36",
  "term_id": "UNKNOWN:0002",
  "gene": "UniProtKB:Q9H2U1",
  "gene_name": "ATP-dependent DNA_RNA helicase DHX36",
  "term_label": "Unknown biological process"
}